MHC class II protein binding, via antigen binding groove [GO:0042658] (molecular function) Sources: GOC:jl Definition: Binding to the antigen binding groove of major histocompatibility complex class II molecules. Relationships: is a type of GO:0042289; BFO_0000050 MHC class II protein complex binding [GO:0023026] Also known as: major histocompatibility complex class II protein binding, via antigen binding groove